{
  "term_id": "GO:0005737",
  "gene_symbol": "SPATA24",
  "gene": "UniProtKB:Q86W54",
  "term_label": "cytoplasm",
  "gene_name": "Spermatogenesis-associated protein 24"
}